{
  "term_label": "Unknown molecular function",
  "gene": "UniProtKB:O96006",
  "term_id": "UNKNOWN:0001",
  "gene_symbol": "ZBED1",
  "gene_name": "E3 SUMO-protein ligase ZBED1"
}